{
  "gene": "UniProtKB:A0A0B4J1X8",
  "gene_symbol": "IGHV3-43",
  "gene_name": "Immunoglobulin heavy variable 3-43",
  "term_label": "antigen binding",
  "term_id": "GO:0003823"
}